{
  "term_label": "DNA binding",
  "gene_name": "Protein lin-9 homolog",
  "gene_symbol": "LIN9",
  "term_id": "GO:0003677",
  "gene": "UniProtKB:Q5TKA1"
}